{
  "gene_symbol": "PABPC5",
  "gene_name": "Polyadenylate-binding protein 5",
  "term_label": "Unknown biological process",
  "gene": "UniProtKB:Q96DU9",
  "term_id": "UNKNOWN:0002"
}